{
  "term_id": "UNKNOWN:0001",
  "gene_symbol": "TFF1",
  "term_label": "Unknown molecular function",
  "gene_name": "Trefoil factor 1",
  "gene": "UniProtKB:P04155"
}